{
  "gene_symbol": "RRP1B",
  "term_label": "nucleus",
  "term_id": "GO:0005634",
  "gene_name": "Ribosomal RNA processing protein 1 homolog B",
  "gene": "UniProtKB:Q14684"
}